{
  "gene": "UniProtKB:Q9UQK1",
  "term_label": "regulation of glycogen biosynthetic process",
  "gene_name": "Protein phosphatase 1 regulatory subunit 3C",
  "term_id": "GO:0005979",
  "gene_symbol": "PPP1R3C"
}